{
  "gene": "UniProtKB:Q9H1M4",
  "gene_name": "Beta-defensin 127",
  "gene_symbol": "DEFB127",
  "term_label": "Unknown cellular component",
  "term_id": "UNKNOWN:0003"
}